{
  "gene_name": "Uncharacterized protein C20orf203",
  "term_label": "Unknown biological process",
  "term_id": "UNKNOWN:0002",
  "gene": "UniProtKB:Q8NBC4",
  "gene_symbol": "C20orf203"
}